(+)-alpha-barbatene synthase activity [GO:0102878] (molecular function) Definition: Catalysis of the reaction: (2E,6E)-farnesyl diphosphate = (+)-alpha-barbatene + diphosphate. Sources: RHEA:29499 Relationships: is a type of carbon-oxygen lyase activity, acting on phosphates [GO:0016838]